{
  "gene_name": "Interferon alpha-17",
  "gene": "UniProtKB:P01571",
  "gene_symbol": "IFNA17",
  "term_id": "GO:0002286",
  "term_label": "T cell activation involved in immune response"
}